{
  "gene_name": "Tumor necrosis factor receptor superfamily member 16",
  "gene_symbol": "NGFR",
  "term_id": "GO:0009986",
  "term_label": "cell surface",
  "gene": "UniProtKB:P08138"
}